{
  "term_id": "GO:0005788",
  "term_label": "endoplasmic reticulum lumen",
  "gene_name": "Selenoprotein M",
  "gene_symbol": "SELENOM",
  "gene": "UniProtKB:Q8WWX9"
}